{
  "term_label": "semaphorin receptor binding",
  "gene": "UniProtKB:Q9NTN9",
  "gene_name": "Semaphorin-4G",
  "term_id": "GO:0030215",
  "gene_symbol": "SEMA4G"
}